response to resveratrol [GO:1904638] (biological process) Definition: Any process that results in a change in state or activity of a cell or an organism (in terms of movement, secretion, enzyme production, gene expression, etc.) as a result of a resveratrol stimulus. References: PMID:23555824 Sources: GOC:TermGenie, GO_REF:0000071 Relationships: is a type of response to stilbenoid [GO:0035634]; is a type of response to oxygen-containing compound [GO:1901700] Subtypes: GO:1904639